potassium:proton antiporter complex [GO:1903103] (cellular component) References: PMID:21041667 Sources: GOC:TermGenie, GOC:bhm, GO_REF:0000088 Relationships: is a type of GO:1902495 Definition: A protein complex which is capable of potassium:proton antiporter activity. Note: An example of this is kefC in E. coli (P03819) in PMID:21041667 (inferred from direct assay).